{
  "gene_symbol": "STARD9",
  "term_label": "microtubule motor activity",
  "gene_name": "StAR-related lipid transfer protein 9",
  "term_id": "GO:0003777",
  "gene": "UniProtKB:Q9P2P6"
}